{
  "term_label": "cyclin binding",
  "gene_symbol": "KLHDC9",
  "gene": "UniProtKB:Q8NEP7",
  "gene_name": "Kelch domain-containing protein 9",
  "term_id": "GO:0030332"
}